{
  "term_label": "immune receptor activity",
  "gene_name": "Killer cell immunoglobulin-like receptor 3DL3",
  "gene": "UniProtKB:Q8N743",
  "gene_symbol": "KIR3DL3",
  "term_id": "GO:0140375"
}